{
  "term_label": "GTP binding",
  "term_id": "GO:0005525",
  "gene": "UniProtKB:A0A0G2JMH3",
  "gene_symbol": "LOC107984156",
  "gene_name": "ADP-ribosylation factor-like protein 17 C-terminal domain-containing protein"
}